{
  "gene_name": "Putative uncharacterized protein SNHG28",
  "gene": "UniProtKB:P0DPA3",
  "gene_symbol": "SNHG28",
  "term_id": "UNKNOWN:0002",
  "term_label": "Unknown biological process"
}